{
  "term_label": "RNA polymerase II cis-regulatory region sequence-specific DNA binding",
  "term_id": "GO:0000978",
  "gene_symbol": "VENTX",
  "gene_name": "Homeobox protein VENTX",
  "gene": "UniProtKB:O95231"
}